N-acylglucosamine-6-phosphate 2-epimerase activity [GO:0047465] (molecular function) Relationships: is a type of racemase and epimerase activity, acting on carbohydrates and derivatives [GO:0016857] Also known as: N-acetylglucosmamine 6-phosphate 2-epimerase activity, N-acetylmannosamine-6-phosphate 2-epimerase activity, N-acyl-D-glucosamine-6-phosphate 2-epimerase activity, acylglucosamine phosphate 2-epimerase activity, acylglucosamine-6-phosphate 2-epimerase activity, acylmannosamine phosphate 2-epimerase activity Definition: Catalysis of the reaction: an N-acyl-D-glucosamine 6-phosphate = an N-acyl-D-mannosamine 6-phosphate. Sources: RHEA:23932